viral procapsid [GO:0046729] (cellular component) Sources: ISBN:0072370319, ISBN:1555811272 Definition: A stable empty viral capsid produced during the assembly of viruses. Relationships: is a type of virion component [GO:0044423]